galactose-1-phosphate phosphatase activity [GO:0070456] (molecular function) Subtypes: L-galactose-1-phosphate phosphatase activity [GO:0010347], D-galactose-1-phosphate phosphatase activity [GO:0070457] Relationships: is a type of GO:0050308 Definition: Catalysis of the reaction: galactose-1-phosphate + H2O = galactose + phosphate. Sources: GOC:mah